D-lyxose ketol-isomerase activity [GO:0047828] (molecular function) Relationships: is a type of intramolecular oxidoreductase activity, interconverting aldoses and ketoses [GO:0016861] Sources: EC:5.3.1.15, RHEA:14201 Definition: Catalysis of the reaction: D-lyxose = D-xylulose. Also known as: D-lyxose aldose-ketose-isomerase activity, D-lyxose isomerase activity